morphogenesis of a branching structure [GO:0001763] (biological process) Relationships: is a type of anatomical structure morphogenesis [GO:0009653]; is a type of GO:0032501 Subtypes: GO:0010223, GO:0048755, morphogenesis of a branching epithelium [GO:0061138], lateral root branching [GO:0080181] Sources: ISBN:0721662544 Definition: The process in which the anatomical structures of branches are generated and organized. A branch is a division or offshoot from a main stem. Examples in animals would include blood vessels, nerves, lymphatics and other endothelial or epithelial tubes. Also known as: branching morphogenesis Regulation: regulated by GO:0060688